(S)-stylopine synthase activity [GO:0047052] (molecular function) Also known as: (S)-cheilanthifoline oxidase (methylenedioxy-bridge-forming) activity, (S)-cheilanthifoline,NADPH:oxygen oxidoreductase (methylenedioxy-bridge-forming) Definition: Catalysis of the reaction: (S)-cheilanthifoline + reduced [NADPH--hemoprotein reductase] + O2 = (S)-stylopine + oxidized [NADPH--hemoprotein reductase] + 2 H2O + H+. Sources: RHEA:13773 Relationships: is a type of oxidoreductase activity, acting on paired donors, with oxidation of a pair of donors resulting in the reduction of molecular oxygen to two molecules of water [GO:0016717]